{
  "gene_symbol": "JPT2",
  "gene_name": "Jupiter microtubule associated homolog 2",
  "gene": "UniProtKB:Q9H910",
  "term_id": "GO:0005634",
  "term_label": "nucleus"
}